{
  "term_id": "GO:0098978",
  "gene_symbol": "DGKI",
  "gene": "UniProtKB:O75912",
  "gene_name": "Diacylglycerol kinase iota",
  "term_label": "glutamatergic synapse"
}